{
  "gene_name": "Calmodulin-like protein 4",
  "term_id": "GO:0030234",
  "gene_symbol": "CALML4",
  "term_label": "enzyme regulator activity",
  "gene": "UniProtKB:Q96GE6"
}